{
  "gene": "UniProtKB:Q9UKD1",
  "gene_name": "Glucocorticoid modulatory element-binding protein 2",
  "term_label": "RNA polymerase II cis-regulatory region sequence-specific DNA binding",
  "term_id": "GO:0000978",
  "gene_symbol": "GMEB2"
}